{
  "gene_name": "Calcium and integrin-binding family member 2",
  "term_id": "GO:0055074",
  "gene": "UniProtKB:O75838",
  "term_label": "calcium ion homeostasis",
  "gene_symbol": "CIB2"
}